cellular response to L-arginine [GO:1903577] (biological process) Relationships: is a type of GO:0071230; is a type of cellular response to nitrogen compound [GO:1901699]; is a type of cellular response to oxygen-containing compound [GO:1901701]; is a type of response to L-arginine [GO:1903576] Definition: Any process that results in a change in state or activity of a cell (in terms of movement, secretion, enzyme production, gene expression, etc.) as a result of a L-arginine stimulus. References: PMID:6394628 Sources: GOC:TermGenie, GOC:mr, GO_REF:0000071